{
  "gene_symbol": "MEN1",
  "gene_name": "Menin",
  "term_id": "GO:0008285",
  "gene": "UniProtKB:O00255",
  "term_label": "negative regulation of cell population proliferation"
}